{
  "term_label": "calcium ion sensor activity",
  "gene_name": "EF-hand domain-containing family member B",
  "term_id": "GO:0061891",
  "gene": "UniProtKB:Q8N7U6",
  "gene_symbol": "EFHB"
}